{
  "gene": "UniProtKB:P15923",
  "term_label": "DNA-binding transcription factor activity, RNA polymerase II-specific",
  "gene_name": "Transcription factor E2-alpha",
  "term_id": "GO:0000981",
  "gene_symbol": "TCF3"
}